{
  "term_label": "plasma membrane",
  "gene_symbol": "RHAG",
  "term_id": "GO:0005886",
  "gene": "UniProtKB:Q02094",
  "gene_name": "Ammonium transporter Rh type A"
}